geranyl diphosphate metabolic process [GO:0033383] (biological process) Definition: The chemical reactions and pathways involving geranyl diphosphate, the universal precursor of the monoterpenes. Subtypes: geranyl diphosphate biosynthetic process [GO:0033384] Also known as: geranyl diphosphate metabolism, geranyldiphosphate metabolic process Relationships: is a type of phospholipid metabolic process [GO:0006644]; is a type of terpenoid metabolic process [GO:0006721] Sources: GOC:mah